{
  "term_id": "GO:0004045",
  "gene_name": "Peptidyl-tRNA hydrolase 2, mitochondrial",
  "gene": "UniProtKB:Q9Y3E5",
  "gene_symbol": "PTRH2",
  "term_label": "peptidyl-tRNA hydrolase activity"
}